{
  "gene": "UniProtKB:Q9UQF0",
  "term_id": "UNKNOWN:0003",
  "gene_symbol": "ERVW-1",
  "term_label": "Unknown cellular component",
  "gene_name": "Syncytin-1"
}